{
  "gene_name": "Sodium-coupled neutral amino acid transporter 4",
  "term_label": "L-amino acid transmembrane transporter activity",
  "gene_symbol": "SLC38A4",
  "gene": "UniProtKB:Q969I6",
  "term_id": "GO:0015179"
}